{
  "gene_symbol": "GPC1",
  "term_label": "negative regulation of fibroblast growth factor receptor signaling pathway",
  "gene": "UniProtKB:P35052",
  "term_id": "GO:0040037",
  "gene_name": "Glypican-1"
}